{
  "term_id": "GO:0005549",
  "gene_name": "Olfactory receptor 5K4",
  "term_label": "odorant binding",
  "gene_symbol": "OR5K4",
  "gene": "UniProtKB:A6NMS3"
}